protein tyrosine phosphatase activator activity [GO:0008160] (molecular function) Relationships: is a type of protein phosphatase activator activity [GO:0072542]; positively regulates protein tyrosine phosphatase activity [GO:0004725] Sources: GOC:ai, ISBN:0198506732 Definition: Binds to and increases the activity of a phosphotyrosine phosphatase, an enzyme which catalyzes of the removal of a phosphate group from a tyrosyl phenolic group of a protein.